glycine secretion, neurotransmission [GO:0061537] (biological process) Definition: The controlled release of glycine by a cell, in which glycine acts as a neurotransmitter. Relationships: is a type of neurotransmitter secretion [GO:0007269]; is a type of glycine secretion [GO:0061536]; is part of synaptic transmission, glycinergic [GO:0060012] Regulation: regulated by regulation of glycine secretion, neurotransmission [GO:1904624]; negatively regulated by GO:1904625; RO_0002213 by positive regulation of glycine secretion, neurotransmission [GO:1904626] Sources: GOC:dph